{
  "gene_name": "Collagen alpha-1(V) chain",
  "term_label": "collagen fibril organization",
  "gene_symbol": "COL5A1",
  "term_id": "GO:0030199",
  "gene": "UniProtKB:P20908"
}